{
  "gene": "UniProtKB:P49721",
  "gene_name": "Proteasome subunit beta type-2",
  "term_id": "GO:0005829",
  "term_label": "cytosol",
  "gene_symbol": "PSMB2"
}